{
  "term_label": "Unknown molecular function",
  "gene_name": "Guanine nucleotide exchange factor subunit RIC1",
  "gene": "UniProtKB:Q4ADV7",
  "gene_symbol": "RIC1",
  "term_id": "UNKNOWN:0001"
}